{
  "term_id": "GO:0071277",
  "gene_name": "Adhesion G-protein coupled receptor V1",
  "gene_symbol": "ADGRV1",
  "term_label": "cellular response to calcium ion",
  "gene": "UniProtKB:Q8WXG9"
}